{
  "gene": "UniProtKB:P10909",
  "term_label": "misfolded protein binding",
  "gene_symbol": "CLU",
  "gene_name": "Clusterin",
  "term_id": "GO:0051787"
}